{
  "gene": "UniProtKB:P63000",
  "gene_name": "Ras-related C3 botulinum toxin substrate 1",
  "gene_symbol": "RAC1",
  "term_label": "cell projection",
  "term_id": "GO:0042995"
}